{
  "gene": "UniProtKB:Q9Y274",
  "gene_symbol": "ST3GAL6",
  "term_id": "GO:0009247",
  "gene_name": "Type 2 lactosamine alpha-2,3-sialyltransferase",
  "term_label": "glycolipid biosynthetic process"
}